plasma membrane [GO:0005886] (cellular component) Relationships: is a type of membrane [GO:0016020]; BFO_0000050 GO:0071944 Also known as: juxtamembrane, cell membrane, cellular membrane, cytoplasmic membrane, plasmalemma, bacterial inner membrane, inner endospore membrane, integral component of plasma membrane, integral to plasma membrane, plasma membrane lipid bilayer Definition: The membrane surrounding a cell that separates the cell from its external environment. It consists of a phospholipid bilayer and associated proteins. Subtypes: GO:0001533, sarcolemma [GO:0042383], sperm plasma membrane [GO:0097524], apical plasma membrane urothelial plaque [GO:0120001] Sources: ISBN:0716731363